{
  "term_label": "mRNA binding",
  "gene_name": "Cleavage and polyadenylation specificity factor subunit 6",
  "gene_symbol": "CPSF6",
  "gene": "UniProtKB:Q16630",
  "term_id": "GO:0003729"
}